{
  "term_label": "Unknown molecular function",
  "gene": "UniProtKB:Q86WR0",
  "gene_name": "Coiled-coil domain-containing protein 25",
  "term_id": "UNKNOWN:0001",
  "gene_symbol": "CCDC25"
}